{
  "gene_name": "Protein Dr1",
  "term_id": "GO:0017054",
  "gene_symbol": "DR1",
  "term_label": "negative cofactor 2 complex",
  "gene": "UniProtKB:Q01658"
}